{
  "term_id": "GO:0000127",
  "term_label": "transcription factor TFIIIC complex",
  "gene": "UniProtKB:Q969F1",
  "gene_name": "General transcription factor 3C polypeptide 6",
  "gene_symbol": "GTF3C6"
}